{
  "gene_name": "Histone H2B type 1-C_E_F_G_I",
  "gene": "UniProtKB:P62807",
  "term_id": "GO:0006325",
  "gene_symbol": "H2BC10",
  "term_label": "chromatin organization"
}